{
  "gene": "UniProtKB:Q96KG7",
  "term_id": "GO:0005112",
  "term_label": "Notch binding",
  "gene_name": "Multiple epidermal growth factor-like domains protein 10",
  "gene_symbol": "MEGF10"
}